{
  "gene": "UniProtKB:Q96IZ0",
  "term_label": "cytoplasm",
  "gene_name": "PRKC apoptosis WT1 regulator protein",
  "gene_symbol": "PAWR",
  "term_id": "GO:0005737"
}